{
  "gene_symbol": "TAS1R3",
  "term_id": "GO:0050916",
  "term_label": "sensory perception of sweet taste",
  "gene": "UniProtKB:Q7RTX0",
  "gene_name": "Taste receptor type 1 member 3"
}